nucleotide-sugar transmembrane transport [GO:0015780] (biological process) Also known as: nucleotide-sugar transport Definition: The directed movement of nucleotide-sugars into, out of or within a cell, or between cells, by means of some agent such as a transporter or pore. Nucleotide-sugars are any nucleotide in which the distal phosphoric residue of a nucleoside 5'-diphosphate is in glycosidic linkage with a monosaccharide or monosaccharide derivative. Sources: ISBN:0198506732 Relationships: is a type of organophosphate ester transport [GO:0015748]; is a type of GO:0015931; is a type of transmembrane transport [GO:0055085]; is a type of carbohydrate derivative transport [GO:1901264] Subtypes: purine nucleotide-sugar transmembrane transport [GO:0090480], pyrimidine nucleotide-sugar transmembrane transport [GO:0090481]